{
  "gene_name": "Glycosylphosphatidylinositol-anchored high density lipoprotein-binding protein 1",
  "term_label": "chylomicron binding",
  "gene": "UniProtKB:Q8IV16",
  "gene_symbol": "GPIHBP1",
  "term_id": "GO:0035478"
}